{
  "term_label": "ubiquitin protein ligase activity",
  "gene": "UniProtKB:Q9H920",
  "gene_symbol": "RNF121",
  "gene_name": "E3 ubiquitin ligase RNF121",
  "term_id": "GO:0061630"
}